phenazine biosynthetic process [GO:0002047] (biological process) Definition: The chemical reactions and pathways resulting in the formation of a phenazine antibiotic, a polycyclic pyrazine with two nitrogen atoms in the ring. Sources: GOC:dph Also known as: acridizine biosynthesis, acridizine biosynthetic process, azophenylene biosynthesis, azophenylene biosynthetic process, dibenzo-p-diazine biosynthesis, dibenzo-p-diazine biosynthetic process, dibenzopyrazine biosynthesis, dibenzopyrazine biosynthetic process Relationships: is a type of antibiotic biosynthetic process [GO:0017000] Regulation: regulated by regulation of phenazine biosynthetic process [GO:1900980]; negatively regulated by negative regulation of phenazine biosynthetic process [GO:1900981]; positively regulated by positive regulation of phenazine biosynthetic process [GO:1900982]